{
  "term_label": "positive regulation of translational initiation",
  "gene": "UniProtKB:Q9NR90",
  "gene_name": "Deleted in azoospermia protein 3",
  "term_id": "GO:0045948",
  "gene_symbol": "DAZ3"
}